cardiac neural crest cell delamination involved in outflow tract morphogenesis [GO:1900728] (biological process) Definition: Any cardiac neural crest cell delamination that is involved in outflow tract morphogenesis. References: PMID:18539270 Sources: GOC:TermGenie, GOC:hjd Relationships: is_a cardiac neural crest cell delamination [GO:0036036]; is part of outflow tract morphogenesis [GO:0003151]